{
  "gene_name": "Guanine nucleotide-binding protein G(t) subunit alpha-3",
  "gene": "UniProtKB:A8MTJ3",
  "term_label": "cytoplasm",
  "gene_symbol": "GNAT3",
  "term_id": "GO:0005737"
}